{
  "term_label": "plasma membrane",
  "term_id": "GO:0005886",
  "gene_symbol": "PIP5K1C",
  "gene": "UniProtKB:O60331",
  "gene_name": "Phosphatidylinositol 4-phosphate 5-kinase type-1 gamma"
}